purine-containing compound catabolic process [GO:0072523] (biological process) Relationships: is a type of catabolic process [GO:0009056]; is a type of purine-containing compound metabolic process [GO:0072521] Subtypes: purine nucleobase catabolic process [GO:0006145], purine nucleoside catabolic process [GO:0006152], purine nucleotide catabolic process [GO:0006195], coenzyme A catabolic process [GO:0015938], GO:0019628, purine nucleoside bisphosphate catabolic process [GO:0034034], GO:0034266, discadenine catabolic process [GO:0034269], GO:0036115, acetyl-CoA catabolic process [GO:0046356], succinyl-CoA catabolic process [GO:1901289], benzoyl-CoA catabolic process [GO:1901788], 2-hydroxybenzoyl-CoA catabolic process [GO:1901886], malonyl-CoA catabolic process [GO:2001294] Also known as: purine and derivative catabolic process, purine-containing compound breakdown, purine-containing compound catabolism, purine-containing compound degradation Definition: The chemical reactions and pathways resulting in the breakdown of a purine-containing compound, i.e. any compound that contains purine or a formal derivative thereof. Sources: GOC:mah